{
  "gene": "UniProtKB:Q9Y5K2",
  "term_id": "GO:0051604",
  "gene_name": "Kallikrein-4",
  "gene_symbol": "KLK4",
  "term_label": "protein maturation"
}